{
  "term_label": "RNA binding",
  "gene_name": "SR-related and CTD-associated factor 4",
  "term_id": "GO:0003723",
  "gene": "UniProtKB:O95104",
  "gene_symbol": "SCAF4"
}